positive regulation of oligodendrocyte differentiation [GO:0048714] (biological process) Relationships: is a type of positive regulation of glial cell differentiation [GO:0045687]; is a type of regulation of oligodendrocyte differentiation [GO:0048713]; positively regulates GO:0048709 Also known as: up regulation of oligodendrocyte differentiation, up-regulation of oligodendrocyte differentiation, upregulation of oligodendrocyte differentiation, activation of oligodendrocyte differentiation, stimulation of oligodendrocyte differentiation References: PMID:15139015 Sources: GOC:vp Definition: Any process that activates or increases the frequency, rate or extent of oligodendrocyte differentiation.